hematopoietic stem cell migration to bone marrow [GO:0097241] (biological process) Also known as: hematopoietic stem cell homing, progenitor cell homing, hemopoietic stem cell migration to bone marrow Relationships: is a type of hematopoietic stem cell migration [GO:0035701] Definition: The orderly movement of a hematopoietic stem cell into the bone marrow, and its subsequent positioning within defined functional compartments in that microenvironment. A hematopoietic stem cell is a cell from which all cells of the lymphoid and myeloid lineages develop, including blood cells and cells of the immune system. References: PMID:17368745 Sources: CL:0000037, GOC:yaf